{
  "gene": "UniProtKB:Q9Y6B6",
  "gene_symbol": "SAR1B",
  "term_label": "COPII vesicle coat",
  "term_id": "GO:0030127",
  "gene_name": "GTP-binding protein SAR1b"
}